{
  "gene": "UniProtKB:Q86UA1",
  "gene_symbol": "PRPF39",
  "gene_name": "Pre-mRNA-processing factor 39",
  "term_label": "U2-type prespliceosome",
  "term_id": "GO:0071004"
}